{
  "gene": "UniProtKB:P62330",
  "term_id": "GO:0055038",
  "term_label": "recycling endosome membrane",
  "gene_symbol": "ARF6",
  "gene_name": "ADP-ribosylation factor 6"
}